{
  "gene": "UniProtKB:P06028",
  "term_id": "UNKNOWN:0002",
  "gene_symbol": "GYPB",
  "term_label": "Unknown biological process",
  "gene_name": "Glycophorin-B"
}